{
  "gene_symbol": "FFAR2",
  "term_id": "GO:0007186",
  "gene_name": "Free fatty acid receptor 2",
  "term_label": "G protein-coupled receptor signaling pathway",
  "gene": "UniProtKB:O15552"
}